{
  "gene_symbol": "HMGB1",
  "term_label": "nucleus",
  "gene_name": "High mobility group protein B1",
  "term_id": "GO:0005634",
  "gene": "UniProtKB:P09429"
}